positive regulation of crystal cell differentiation [GO:0042691] (biological process) Relationships: is a type of regulation of crystal cell differentiation [GO:0042689]; is a type of positive regulation of hemocyte differentiation [GO:0045612]; positively regulates crystal cell differentiation [GO:0042688] Definition: Any process that activates or increases the frequency, rate or extent of crystal cell differentiation. Sources: GOC:go_curators Also known as: up regulation of crystal cell differentiation, up-regulation of crystal cell differentiation, upregulation of crystal cell differentiation, activation of crystal cell differentiation, stimulation of crystal cell differentiation